{
  "term_id": "GO:0007186",
  "gene": "UniProtKB:Q8NGL2",
  "term_label": "G protein-coupled receptor signaling pathway",
  "gene_name": "Olfactory receptor 5L1",
  "gene_symbol": "OR5L1"
}